{
  "term_id": "GO:0005938",
  "gene_name": "Partitioning defective 3 homolog",
  "term_label": "cell cortex",
  "gene": "UniProtKB:Q8TEW0",
  "gene_symbol": "PARD3"
}